{
  "term_id": "GO:0090263",
  "gene": "UniProtKB:Q2I0M5",
  "gene_symbol": "RSPO4",
  "term_label": "positive regulation of canonical Wnt signaling pathway",
  "gene_name": "R-spondin-4"
}